ceramide kinase activity [GO:0001729] (molecular function) Also known as: ATP:ceramide 1-phosphotransferase activity, acylsphingosine kinase activity Sources: EC:2.7.1.138 Relationships: is a type of lipid kinase activity [GO:0001727] Definition: Catalysis of the reaction: an N-acylsphing-4-enine + ATP = ADP + an N-acylsphing-4-enine 1-phosphate + H+.